{
  "gene": "UniProtKB:P61962",
  "term_id": "GO:0005634",
  "gene_name": "DDB1- and CUL4-associated factor 7",
  "term_label": "nucleus",
  "gene_symbol": "DCAF7"
}